{
  "gene_symbol": "RHPN1-AS1",
  "term_id": "UNKNOWN:0003",
  "gene": "UniProtKB:Q9BWJ2",
  "term_label": "Unknown cellular component",
  "gene_name": "Putative uncharacterized protein encoded by RHPN1-AS1"
}